phenyl propionate uniporter activity [GO:0015544] (MF) Definition: Enables the transfer of phenyl propionate from one side of a membrane to the other. Sources: GOC:mtg_transport, TC:2.A.1.27.1 Also known as: phenyl propionate permease activity Relationships: is a type of uniporter activity [GO:0015292]; is a type of secondary active monocarboxylate transmembrane transporter activity [GO:0015355]; is a type of propionate transmembrane transporter activity [GO:0015552]